{
  "term_label": "cytoplasm",
  "gene_symbol": "MC4R",
  "gene_name": "Melanocortin receptor 4",
  "gene": "UniProtKB:P32245",
  "term_id": "GO:0005737"
}